{
  "gene": "UniProtKB:Q2NKX9",
  "gene_name": "UPF0561 protein C2orf68",
  "term_id": "UNKNOWN:0001",
  "gene_symbol": "C2orf68",
  "term_label": "Unknown molecular function"
}